{
  "term_id": "GO:0048066",
  "term_label": "developmental pigmentation",
  "gene_symbol": "HPS5",
  "gene_name": "BLOC-2 complex member HPS5",
  "gene": "UniProtKB:Q9UPZ3"
}